{
  "gene": "UniProtKB:Q8WTR8",
  "term_label": "substrate adhesion-dependent cell spreading",
  "term_id": "GO:0034446",
  "gene_symbol": "NTN5",
  "gene_name": "Netrin-5"
}